{
  "gene": "UniProtKB:Q9BYC8",
  "term_label": "mitochondrial large ribosomal subunit",
  "gene_symbol": "MRPL32",
  "gene_name": "Large ribosomal subunit protein bL32m",
  "term_id": "GO:0005762"
}